{
  "gene_name": "Gamma-aminobutyric acid receptor subunit alpha-5",
  "gene_symbol": "GABRA5",
  "term_id": "GO:0008503",
  "gene": "UniProtKB:P31644",
  "term_label": "benzodiazepine receptor activity"
}